{
  "gene": "UniProtKB:Q9P0W0",
  "gene_symbol": "IFNK",
  "term_id": "GO:0002250",
  "gene_name": "Interferon kappa",
  "term_label": "adaptive immune response"
}